{
  "term_label": "Unknown biological process",
  "gene_name": "Ankyrin repeat domain-containing protein 50",
  "term_id": "UNKNOWN:0002",
  "gene_symbol": "ANKRD50",
  "gene": "UniProtKB:Q9ULJ7"
}